{
  "gene": "UniProtKB:Q13296",
  "term_id": "GO:0005615",
  "gene_name": "Mammaglobin-A",
  "term_label": "extracellular space",
  "gene_symbol": "SCGB2A2"
}